2-hexadecenal reductase activity [GO:0047543] (molecular function) Definition: Catalysis of the reaction: NADP+ + palmitaldehyde = trans-hexadec-2-enal + H+ + NADPH. Relationships: is a type of oxidoreductase activity, acting on the CH-CH group of donors, NAD or NADP as acceptor [GO:0016628] Sources: EC:1.3.1.27, RHEA:12444 Also known as: hexadecanal: NADP+ oxidoreductase activity, hexadecanal:NADP+ delta2-oxidoreductase activity